{
  "gene": "UniProtKB:Q9NPH6",
  "term_label": "extracellular space",
  "term_id": "GO:0005615",
  "gene_name": "Odorant-binding protein 2b",
  "gene_symbol": "OBP2B"
}